{
  "gene_name": "Fibroblast growth factor receptor 3",
  "term_id": "GO:0008284",
  "gene": "UniProtKB:P22607",
  "term_label": "positive regulation of cell population proliferation",
  "gene_symbol": "FGFR3"
}